indole-containing compound catabolic process [GO:0042436] (BP) Definition: The chemical reactions and pathways resulting in the breakdown of compounds that contain an indole (2,3-benzopyrrole) skeleton. Sources: GOC:jl Also known as: indole derivative catabolic process, indole derivative catabolism, indole-containing compound breakdown, indole-containing compound catabolism, indole-containing compound degradation Relationships: is a type of catabolic process [GO:0009056]; is a type of indole-containing compound metabolic process [GO:0042430] Subtypes: L-tryptophan catabolic process [GO:0006569], indole glucosinolate catabolic process [GO:0042344], GO:0042429, indole catabolic process [GO:0042433], GO:0042437, melatonin catabolic process [GO:0042442], indole phytoalexin catabolic process [GO:0046216]